{
  "gene_name": "Kelch-like protein 1",
  "term_id": "GO:0005737",
  "gene_symbol": "KLHL1",
  "term_label": "cytoplasm",
  "gene": "UniProtKB:Q9NR64"
}